{
  "gene_symbol": "MNT",
  "gene": "UniProtKB:Q99583",
  "term_id": "UNKNOWN:0003",
  "gene_name": "Max-binding protein MNT",
  "term_label": "Unknown cellular component"
}